{
  "gene_symbol": "NUTM2E",
  "gene_name": "NUT family member 2E",
  "term_id": "UNKNOWN:0003",
  "term_label": "Unknown cellular component",
  "gene": "UniProtKB:B1AL46"
}